{
  "gene_symbol": "FXYD1",
  "term_id": "UNKNOWN:0003",
  "gene": "UniProtKB:O00168",
  "gene_name": "Phospholemman",
  "term_label": "Unknown cellular component"
}